{
  "term_id": "UNKNOWN:0001",
  "gene": "UniProtKB:A6NIJ5",
  "gene_name": "Putative protein FAM90A20P",
  "gene_symbol": "FAM90A20P",
  "term_label": "Unknown molecular function"
}